{
  "gene": "UniProtKB:O14512",
  "term_id": "GO:0008286",
  "term_label": "insulin receptor signaling pathway",
  "gene_symbol": "SOCS7",
  "gene_name": "Suppressor of cytokine signaling 7"
}